{
  "gene_symbol": "NAA35",
  "gene_name": "N-alpha-acetyltransferase 35, NatC auxiliary subunit",
  "term_label": "NatC complex",
  "gene": "UniProtKB:Q5VZE5",
  "term_id": "GO:0031417"
}